{
  "gene": "UniProtKB:Q8NGN4",
  "gene_name": "Olfactory receptor 10G9",
  "term_id": "GO:0004984",
  "gene_symbol": "OR10G9",
  "term_label": "olfactory receptor activity"
}